{
  "term_label": "trans-Golgi network",
  "gene_name": "Ras-related protein Rab-38",
  "term_id": "GO:0005802",
  "gene_symbol": "RAB38",
  "gene": "UniProtKB:P57729"
}